{
  "term_label": "Unknown molecular function",
  "term_id": "UNKNOWN:0001",
  "gene_symbol": "CCL20",
  "gene": "UniProtKB:P78556",
  "gene_name": "C-C motif chemokine 20"
}